{
  "gene_name": "Large ribosomal subunit protein eL28",
  "term_id": "UNKNOWN:0001",
  "term_label": "Unknown molecular function",
  "gene_symbol": "RPL28",
  "gene": "UniProtKB:P46779"
}